regulation of G protein-coupled receptor internalization [GO:1904020] (biological process) Definition: Any process that modulates the frequency, rate or extent of G protein-coupled receptor internalization. Relationships: is a type of regulation of receptor internalization [GO:0002090]; is a type of GO:0008277; regulates G protein-coupled receptor internalization [GO:0002031] Subtypes: negative regulation of G protein-coupled receptor internalization [GO:1904021], GO:1904022 References: PMID:24732013 Sources: GOC:TermGenie, GO_REF:0000058 Also known as: regulation of G-protein-coupled receptor internalization